{
  "term_id": "GO:0071013",
  "gene": "UniProtKB:Q15459",
  "gene_name": "Splicing factor 3A subunit 1",
  "term_label": "catalytic step 2 spliceosome",
  "gene_symbol": "SF3A1"
}